negative regulation of ventricular cardiac muscle cell action potential [GO:1903946] (biological process) Definition: Any process that stops, prevents or reduces the frequency, rate or extent of ventricular cardiac muscle cell action potential. References: PMID:25281747 Sources: GOC:BHF, GOC:TermGenie, GOC:mtg_cardiac_conduct_nov11, GOC:nc, GO_REF:0000058 Relationships: is_a negative regulation of action potential [GO:0045759]; is a type of regulation of ventricular cardiac muscle cell action potential [GO:0098911]; is a type of negative regulation of cardiac muscle cell contraction [GO:0106135]; negatively regulates ventricular cardiac muscle cell action potential [GO:0086005] Also known as: down regulation of ventricular cardiac muscle cell action potential, down-regulation of ventricular cardiac muscle cell action potential, downregulation of ventricular cardiac muscle cell action potential, inhibition of ventricular cardiac muscle cell action potential